{
  "gene_symbol": "GTPBP3",
  "term_id": "GO:0005737",
  "term_label": "cytoplasm",
  "gene_name": "tRNA modification GTPase GTPBP3, mitochondrial",
  "gene": "UniProtKB:Q969Y2"
}